{
  "gene_name": "NADH dehydrogenase [ubiquinone] flavoprotein 1, mitochondrial",
  "gene": "UniProtKB:P49821",
  "term_label": "respiratory chain complex I",
  "term_id": "GO:0045271",
  "gene_symbol": "NDUFV1"
}